{
  "gene": "UniProtKB:O43854",
  "gene_name": "EGF-like repeat and discoidin I-like domain-containing protein 3",
  "term_label": "extracellular space",
  "gene_symbol": "EDIL3",
  "term_id": "GO:0005615"
}